{
  "term_label": "cytoplasm",
  "term_id": "GO:0005737",
  "gene_name": "Serine_threonine-protein kinase 11-interacting protein",
  "gene_symbol": "STK11IP",
  "gene": "UniProtKB:Q8N1F8"
}